{
  "gene": "UniProtKB:Q86V21",
  "gene_name": "Acetoacetyl-CoA synthetase",
  "term_label": "Unknown cellular component",
  "gene_symbol": "AACS",
  "term_id": "UNKNOWN:0003"
}